{
  "gene_symbol": "AEN",
  "gene": "UniProtKB:Q8WTP8",
  "term_id": "GO:0005634",
  "term_label": "nucleus",
  "gene_name": "Apoptosis-enhancing nuclease"
}